{
  "gene_symbol": "KCNA7",
  "gene": "UniProtKB:Q96RP8",
  "term_label": "membrane",
  "gene_name": "Potassium voltage-gated channel subfamily A member 7",
  "term_id": "GO:0016020"
}